neopullulanase activity [GO:0031216] (molecular function) Also known as: pullulanase II activity, pullulan 4-D-glucanohydrolase (panose-forming) Definition: Catalysis of the hydrolysis of pullulan to panose (6-alpha-D-glucosylmaltose). Sources: EC:3.2.1.135, GOC:mlg Relationships: is a type of hydrolase activity, hydrolyzing O-glycosyl compounds [GO:0004553]